{
  "gene": "UniProtKB:A0A087X096",
  "gene_symbol": "TRAJ37",
  "term_label": "Unknown molecular function",
  "term_id": "UNKNOWN:0001",
  "gene_name": "T cell receptor alpha joining 37 (Fragment)"
}